{
  "term_id": "GO:0005737",
  "gene": "UniProtKB:P23219",
  "gene_name": "Prostaglandin G_H synthase 1",
  "gene_symbol": "PTGS1",
  "term_label": "cytoplasm"
}